{
  "term_id": "GO:0016064",
  "gene_name": "Immunoglobulin heavy variable 3-30",
  "term_label": "immunoglobulin mediated immune response",
  "gene_symbol": "IGHV3-30",
  "gene": "UniProtKB:P01768"
}